vesicle fusion with Golgi cis cisterna membrane [GO:1990670] (biological process) Relationships: is a type of GO:0006906 References: PMID:16038056, PMID:24119662 Sources: GOC:bhm Subtypes: endoplasmic reticulum-Golgi intermediate compartment (ERGIC) derived vesicle fusion with Golgi cis cisterna membrane [GO:1990689] Definition: The joining of the lipid bilayer membrane around a vesicle to the lipid bilayer membrane around the Golgi cis cisterna. This can involve anterograde or retrograde transport vesicles.